purine nucleotide import into lysosome [GO:0141013] (biological process) Relationships: is a type of lysosomal transport [GO:0007041]; is a type of vacuolar transmembrane transport [GO:0034486]; is a type of purine-containing compound transmembrane transport [GO:0072530] References: PMID:18375752, PMID:23876310 Definition: The directed import of purine nucleotide from the cytosol, across the lysosomal membrane, into the lysosome.